N-glycolylneuraminic acid (Neu5Gc) cytidylyltransferase activity [GO:0090632] (molecular function) Definition: Catalysis of the reaction: CTP + Neu5Gc = diphosphate + CMP-Neu5Gc. References: PMID:11479279, PMID:8381411 Sources: ISBN:978-1-60805-067-3 Also known as: CMP-Neu5Gc synthetase activity Relationships: is_a GO:0070567